{
  "gene_name": "Humanin-like 5",
  "term_id": "UNKNOWN:0003",
  "term_label": "Unknown cellular component",
  "gene": "UniProtKB:P0CJ72",
  "gene_symbol": "MTRNR2L5"
}